{
  "term_label": "Unknown molecular function",
  "gene": "UniProtKB:Q01629",
  "gene_name": "Interferon-induced transmembrane protein 2",
  "gene_symbol": "IFITM2",
  "term_id": "UNKNOWN:0001"
}